{
  "gene_name": "Wee1-like protein kinase",
  "gene_symbol": "WEE1",
  "term_id": "GO:0005634",
  "gene": "UniProtKB:P30291",
  "term_label": "nucleus"
}